{
  "gene_symbol": "ZNF98",
  "gene": "UniProtKB:A6NK75",
  "term_label": "Unknown cellular component",
  "term_id": "UNKNOWN:0003",
  "gene_name": "Zinc finger protein 98"
}